{
  "gene": "UniProtKB:Q9Y5Q6",
  "term_id": "GO:0001664",
  "term_label": "G protein-coupled receptor binding",
  "gene_name": "Insulin-like peptide INSL5",
  "gene_symbol": "INSL5"
}